{
  "gene_name": "Uncharacterized protein C17orf100",
  "gene_symbol": "C17orf100",
  "gene": "UniProtKB:A8MU93",
  "term_label": "Unknown biological process",
  "term_id": "UNKNOWN:0002"
}